{
  "term_label": "serine-type endopeptidase activity",
  "gene_name": "Serine protease HTRA1",
  "gene_symbol": "HTRA1",
  "term_id": "GO:0004252",
  "gene": "UniProtKB:Q92743"
}